{
  "gene_name": "Leucine-rich repeat-containing protein 17",
  "term_label": "plasma membrane",
  "gene_symbol": "LRRC17",
  "term_id": "GO:0005886",
  "gene": "UniProtKB:Q8N6Y2"
}